roof of mouth development [GO:0060021] (biological process) Relationships: is a type of anatomical structure development [GO:0048856] Sources: GOC:dph, ISBN:0721662544 Also known as: palatum development Subtypes: secondary palate development [GO:0062009], primitive palate development [GO:0062010], primary palate development [GO:1903929] Definition: The biological process whose specific outcome is the progression of the roof of the mouth from an initial condition to its mature state. This process begins with the formation of the structure and ends with the mature structure. The roof of the mouth is the partition that separates the nasal and oral cavities.